positive regulation of stem cell differentiation [GO:2000738] (biological process) Sources: GOC:obol Definition: Any process that activates or increases the frequency, rate or extent of stem cell differentiation. Subtypes: GO:0051891, positive regulation of hematopoietic stem cell differentiation [GO:1902038], positive regulation of neural crest cell differentiation [GO:1905294], GO:2000741 Relationships: is a type of positive regulation of cell differentiation [GO:0045597]; is_a regulation of stem cell differentiation [GO:2000736]; positively regulates GO:0048863